{
  "gene_name": "Testis-expressed protein 44",
  "term_id": "UNKNOWN:0002",
  "term_label": "Unknown biological process",
  "gene_symbol": "TEX44",
  "gene": "UniProtKB:Q53QW1"
}